{
  "gene": "UniProtKB:Q86X59",
  "term_label": "Unknown biological process",
  "gene_symbol": "LINC02875",
  "gene_name": "Putative uncharacterized protein LINC02875",
  "term_id": "UNKNOWN:0002"
}